negative regulation of cellular response to alcohol [GO:1905958] (biological process) Definition: Any process that stops, prevents or reduces the frequency, rate or extent of cellular response to alcohol. Subtypes: GO:0009788, negative regulation of ecdysone receptor signaling pathway [GO:0120143] References: PMID:26434723 Sources: GOC:TermGenie, GO_REF:0000058 Also known as: down regulation of cellular response to alcohol, down-regulation of cellular response to alcohol, downregulation of cellular response to alcohol, inhibition of cellular response to alcohol Relationships: is_a negative regulation of cellular process [GO:0048523]; is a type of GO:1901420; is a type of regulation of cellular response to alcohol [GO:1905957]; negatively regulates cellular response to alcohol [GO:0097306]